negative regulation of mRNA modification [GO:0090367] (biological process) Definition: Any process that decreases the rate, frequency, or extent of the covalent alteration of one or more nucleotides within an mRNA molecule to produce an mRNA molecule with a sequence that differs from that coded genetically. Sources: GOC:dph, GOC:sl, GOC:tb Relationships: is a type of regulation of mRNA modification [GO:0090365]; is a type of GO:1903312; negatively regulates mRNA modification [GO:0016556]